BAK complex [GO:0097145] (cellular component) Relationships: is_a GO:0097136 Definition: An oligomeric protein complex consisting of BAK, a member of the Bcl-2 family of anti- and proapoptotic regulators. References: PMID:14634621 Sources: GOC:so